{
  "term_label": "plasma membrane",
  "gene_symbol": "ERBB2",
  "term_id": "GO:0005886",
  "gene_name": "Receptor tyrosine-protein kinase erbB-2",
  "gene": "UniProtKB:P04626"
}